photoreceptor cell morphogenesis [GO:0008594] (biological process) Definition: The process in which the structures of a photoreceptor cell are generated and organized. This process occurs while the initially relatively unspecialized cell is acquiring the specialized features of a photoreceptor cell, a sensory cell that reacts to the presence of light. An example of this is found in Drosophila melanogaster. Sources: GOC:jid, GOC:mah Also known as: photoreceptor development Relationships: is a type of cell morphogenesis involved in neuron differentiation [GO:0048667]; is part of photoreceptor cell development [GO:0042461]